{
  "gene": "UniProtKB:Q9Y2U9",
  "gene_symbol": "KLHDC2",
  "term_label": "Unknown molecular function",
  "gene_name": "Kelch domain-containing protein 2",
  "term_id": "UNKNOWN:0001"
}